{
  "gene": "UniProtKB:Q96P09",
  "term_label": "cysteine-type endopeptidase inhibitor activity involved in apoptotic process",
  "term_id": "GO:0043027",
  "gene_symbol": "BIRC8",
  "gene_name": "Baculoviral IAP repeat-containing protein 8"
}